{
  "gene_symbol": "ZNF687",
  "term_label": "Unknown biological process",
  "gene_name": "Zinc finger protein 687",
  "gene": "UniProtKB:Q8N1G0",
  "term_id": "UNKNOWN:0002"
}